homeostasis of number of cells within a tissue [GO:0048873] (biological process) Definition: Any biological process involved in the maintenance of the steady-state number of cells within a population of cells in a tissue. Relationships: is a type of tissue homeostasis [GO:0001894]; is a type of GO:0048872 Subtypes: homeostasis of number of meristem cells [GO:0007639], homeostasis of number of retina cells [GO:0048877] Sources: GOC:isa_complete